{
  "gene_name": "Late cornified envelope protein 1D",
  "gene": "UniProtKB:Q5T752",
  "term_id": "UNKNOWN:0003",
  "term_label": "Unknown cellular component",
  "gene_symbol": "LCE1D"
}